{
  "gene_name": "Sodium_potassium_calcium exchanger 2",
  "term_id": "GO:0008273",
  "gene_symbol": "SLC24A2",
  "gene": "UniProtKB:Q9UI40",
  "term_label": "calcium, potassium:sodium antiporter activity"
}